{
  "term_label": "lysosomal membrane",
  "term_id": "GO:0005765",
  "gene": "UniProtKB:Q6ZP29",
  "gene_name": "Lysosomal amino acid transporter 1 homolog",
  "gene_symbol": "SLC66A1"
}